{
  "gene": "UniProtKB:Q14592",
  "gene_symbol": "ZNF460",
  "gene_name": "Zinc finger protein 460",
  "term_label": "DNA-binding transcription factor activity, RNA polymerase II-specific",
  "term_id": "GO:0000981"
}